{
  "gene_name": "Acetylcholine receptor subunit epsilon",
  "term_label": "chemical synaptic transmission",
  "gene": "UniProtKB:Q04844",
  "gene_symbol": "CHRNE",
  "term_id": "GO:0007268"
}